{
  "term_label": "Unknown molecular function",
  "term_id": "UNKNOWN:0001",
  "gene_symbol": "BCAS2",
  "gene_name": "Pre-mRNA-splicing factor SPF27",
  "gene": "UniProtKB:O75934"
}